{
  "gene": "UniProtKB:P55072",
  "gene_name": "Transitional endoplasmic reticulum ATPase",
  "term_id": "GO:0034098",
  "gene_symbol": "VCP",
  "term_label": "VCP-NPL4-UFD1 AAA ATPase complex"
}